arabinan endo-1,5-alpha-L-arabinosidase activity [GO:0046558] (molecular function) Also known as: 1,5-alpha-L-arabinan 1,5-alpha-L-arabinanohydrolase activity, endo-1,5-alpha-L-arabinanase activity, endo-alpha-1,5-arabanase activity, endo-arabanase activity Definition: Catalysis of the endohydrolysis of (1->5)-alpha-arabinofuranosidic linkages in (1->5) arabinans. Relationships: is a type of GO:0004553 Sources: EC:3.2.1.99